gut granule [GO:0044840] (cellular component) Definition: A lysosome-related organelle contained within the intestinal cells of the nematode C. elegans. Gut granules are acidified, birefringent, autofluorescent, and contain the vacuolar H+-ATPase. They also serve as sites of cellular zinc storage. References: PMID:22916203, PMID:24204312 Sources: GOC:kmv Relationships: is a type of cytoplasmic vesicle [GO:0031410]